pyridoxine 5-dehydrogenase activity [GO:0050238] (molecular function) Definition: Catalysis of the reaction: pyridoxine + acceptor = isopyridoxal + reduced acceptor. Sources: EC:1.1.99.9, MetaCyc:PYRIDOXINE-5-DEHYDROGENASE-RXN Relationships: is a type of oxidoreductase activity, acting on CH-OH group of donors [GO:0016614] Also known as: pyridoxal-5-dehydrogenase activity, pyridoxin 5-dehydrogenase activity, pyridoxine 5'-dehydrogenase activity, pyridoxine:(acceptor) 5-oxidoreductase activity, pyridoxine:acceptor 5-oxidoreductase activity, pyridoxol 5-dehydrogenase activity